{
  "gene_name": "Transcription factor Spi-C",
  "term_label": "DNA-binding transcription factor activity, RNA polymerase II-specific",
  "gene": "UniProtKB:Q8N5J4",
  "gene_symbol": "SPIC",
  "term_id": "GO:0000981"
}